{
  "term_id": "GO:0004930",
  "term_label": "G protein-coupled receptor activity",
  "gene_name": "Probable G-protein coupled receptor 150",
  "gene_symbol": "GPR150",
  "gene": "UniProtKB:Q8NGU9"
}